{
  "gene_name": "FYN-binding protein 1",
  "term_label": "integrin-mediated signaling pathway",
  "gene_symbol": "FYB1",
  "gene": "UniProtKB:O15117",
  "term_id": "GO:0007229"
}